regulation of centriole elongation [GO:1903722] (biological process) Relationships: is a type of regulation of cell cycle process [GO:0010564]; regulates centriole elongation [GO:0061511] References: PMID:20616062 Sources: GOC:TermGenie, GOC:als, GO_REF:0000058 Definition: Any process that modulates the frequency, rate or extent of centriole elongation. Subtypes: negative regulation of centriole elongation [GO:1903723], positive regulation of centriole elongation [GO:1903724]